plus-end directed microfilament motor activity [GO:0060002] (molecular function) References: PMID:10519557 Sources: GOC:dph Relationships: is a type of microfilament motor activity [GO:0000146] Definition: A motor activity that generates movement along a microfilament towards the plus end, driven by ATP hydrolysis. The minus end of an actin filament is the end that does not preferentially add actin monomers. Also known as: barbed-end directed actin-filament motor activity, plus-end directed actin-filament motor activity, plus-end directed actin filament motor activity